{
  "term_label": "transmembrane-ephrin receptor activity",
  "gene_name": "Ephrin type-B receptor 3",
  "gene_symbol": "EPHB3",
  "term_id": "GO:0005005",
  "gene": "UniProtKB:P54753"
}